viral release from host cell [GO:0019076] (biological process) Definition: The dissemination of mature viral particles from a host cell, e.g. by cell lysis or the budding of virus particles from the cell membrane. Sources: GOC:jl Subtypes: viral release from host cell by cytolysis [GO:0044659], non-lytic viral release [GO:0046753] Relationships: is_a viral process [GO:0016032]; is a type of exit from host cell [GO:0035891]; is part of viral life cycle [GO:0019058] Also known as: release of virus from host, viral exit, viral release, viral shedding, virus exit from host cell